regulation of cellular component size [GO:0032535] (biological process) Relationships: is a type of cellular component organization [GO:0016043]; is a type of regulation of anatomical structure size [GO:0090066] Subtypes: GO:0008361, regulation of myofibril size [GO:0014881], regulation of autophagosome size [GO:0016243], regulation of actin filament length [GO:0030832], regulation of cell projection size [GO:0032536], regulation of translational initiation by eIF2 alpha dephosphorylation [GO:0036496], regulation of peroxisome size [GO:0044375], GO:0062196, regulation of nucleus size [GO:0097298], GO:0097494 Definition: A process that modulates the size of a cellular component. Sources: GOC:mah